{
  "term_id": "UNKNOWN:0001",
  "gene_name": "Leucine-rich repeat-containing protein 66",
  "gene": "UniProtKB:Q68CR7",
  "gene_symbol": "LRRC66",
  "term_label": "Unknown molecular function"
}